{
  "term_label": "Unknown molecular function",
  "term_id": "UNKNOWN:0001",
  "gene_name": "Leucine-rich melanocyte differentiation-associated protein",
  "gene_symbol": "LRMDA",
  "gene": "UniProtKB:Q9H2I8"
}